{
  "gene": "UniProtKB:Q15818",
  "gene_name": "Neuronal pentraxin-1",
  "gene_symbol": "NPTX1",
  "term_id": "UNKNOWN:0001",
  "term_label": "Unknown molecular function"
}